gramicidin S biosynthetic process [GO:1901103] (BP) Relationships: is a type of amide biosynthetic process [GO:0043604] Also known as: gramicidin S anabolism, gramicidin S biosynthesis, gramicidin S formation, gramicidin S synthesis References: PMID:7534306 Sources: GOC:TermGenie, GOC:yaf Definition: The chemical reactions and pathways resulting in the formation of gramicidin S.